{
  "term_label": "Unknown molecular function",
  "gene": "UniProtKB:Q9BV38",
  "gene_symbol": "WDR18",
  "term_id": "UNKNOWN:0001",
  "gene_name": "WD repeat-containing protein 18"
}